{
  "gene_symbol": "FZD5",
  "term_id": "GO:0042813",
  "gene": "UniProtKB:Q13467",
  "gene_name": "Frizzled-5",
  "term_label": "Wnt receptor activity"
}